{
  "term_id": "GO:0030182",
  "gene": "UniProtKB:Q99929",
  "term_label": "neuron differentiation",
  "gene_symbol": "ASCL2",
  "gene_name": "Achaete-scute homolog 2"
}